{
  "gene": "UniProtKB:Q9H5Q4",
  "gene_symbol": "TFB2M",
  "gene_name": "Dimethyladenosine transferase 2, mitochondrial",
  "term_id": "GO:0006391",
  "term_label": "transcription initiation at mitochondrial promoter"
}